lymphocyte migration into lymph node [GO:0097022] (biological process) Definition: The movement of a lymphocyte within the lymphatic system into a lymph node, and its subsequent positioning within defined functional compartments such as sites of cell activation by antigen. Also known as: lymphocyte homing References: PMID:18379575 Sources: GOC:BHF, GOC:pr Relationships: is a type of lymphocyte migration into lymphoid organs [GO:0097021]